small GTPase-mediated signal transduction [GO:0007264] (biological process) Definition: An intracellular signaling cassette in which a small monomeric GTPase relays a signal. Subtypes: GO:0007265, Rho protein signal transduction [GO:0007266], Rac protein signal transduction [GO:0016601], septation initiation signaling [GO:0031028], Ran protein signal transduction [GO:0031291], ARF protein signal transduction [GO:0032011], Rab protein signal transduction [GO:0032482], Ral protein signal transduction [GO:0032484], Rap protein signal transduction [GO:0032486] Relationships: is a type of intracellular signaling cassette [GO:0141124] Regulation: regulated by regulation of small GTPase mediated signal transduction [GO:0051056]; positively regulated by positive regulation of small GTPase mediated signal transduction [GO:0051057]; negatively regulated by GO:0051058 Sources: GOC:mah Also known as: small GTPase mediated signal transduction, Ras family protein signal transduction